{
  "gene": "UniProtKB:Q008S8",
  "term_label": "Unknown molecular function",
  "term_id": "UNKNOWN:0001",
  "gene_symbol": "ECT2L",
  "gene_name": "Epithelial cell-transforming sequence 2 oncogene-like"
}